{
  "gene_symbol": "FEN1",
  "term_label": "nucleus",
  "term_id": "GO:0005634",
  "gene": "UniProtKB:P39748",
  "gene_name": "Flap endonuclease 1"
}